Cdr2 medial cortical node complex [GO:0110115] (cellular component) Definition: A megadalton-sized complex at the medial cortex organized as an oligomeric core of SAD family protein kinases involved in cell size-dependent localization and phosphorylation of Wee1 during interphase. References: PMID:29514920 Sources: GOC:vw Also known as: interphase cortical node, interphase node Relationships: is a type of protein kinase complex [GO:1902911]; BFO_0000050 medial cortical node [GO:0071341]